ribonuclease H2 complex [GO:0032299] (cellular component) Relationships: is a type of intracellular protein-containing complex [GO:0140535]; is a type of catalytic complex [GO:1902494] Also known as: RNase H2 complex References: PMID:14734815 Sources: GOC:mah Definition: A protein complex that possesses ribonuclease H activity, in which the catalytic subunit is a member of the RNase H2 (or HII) class. For example, in Saccharomyces the complex contains Rnh201p, Rnh202p and Rnh203p.